{
  "term_label": "tubulin binding",
  "gene_symbol": "TTLL11",
  "gene": "UniProtKB:Q8NHH1",
  "term_id": "GO:0015631",
  "gene_name": "Tubulin polyglutamylase TTLL11"
}